homoglutathione synthase activity [GO:0047983] (MF) Definition: Catalysis of the reaction: beta-alanine + L-gamma-glutamyl-L-cysteine + ATP = gamma-L-glutamyl-L-cysteinyl-beta-alanine + ADP + 2 H+ + phosphate. Relationships: is a type of acid-amino acid ligase activity [GO:0016881] Also known as: beta-alanine specific hGSH synthetase activity, gamma-L-glutamyl-L-cysteine:beta-alanine ligase (ADP-forming), homoglutathione synthetase activity Sources: EC:6.3.2.23, RHEA:17993